trichloroethene reductive dehalogenase activity [GO:0050697] (molecular function) Sources: RHEA:67992 Also known as: 1,1,2-trichloroethene reductive dehalogenase activity, 1,1,2-trichloroethylene reductive dehalogenase activity, TCE-reductive dehalogenase activity Definition: Catalysis of the reaction: AH2 + trichloroethene = (Z)-1,2-dichloroethene + A + chloride + H+. Relationships: is a type of oxidoreductase activity, acting on X-H and Y-H to form an X-Y bond [GO:0046992]